{
  "gene": "UniProtKB:P10515",
  "term_id": "GO:0045254",
  "gene_symbol": "DLAT",
  "term_label": "pyruvate dehydrogenase complex",
  "gene_name": "Dihydrolipoyllysine-residue acetyltransferase component of pyruvate dehydrogenase complex, mitochondrial"
}